negative regulation of meiotic cell cycle phase transition [GO:1901994] (biological process) Also known as: down regulation of cell cycle transition, down-regulation of cell cycle transition, downregulation of cell cycle transition, inhibition of cell cycle transition, negative regulation of cell cycle transition, down regulation of meiotic cell cycle phase transition, down-regulation of meiotic cell cycle phase transition, downregulation of meiotic cell cycle phase transition, inhibition of meiotic cell cycle phase transition Definition: Any process that stops, prevents or reduces the frequency, rate or extent of meiotic cell cycle phase transition. Subtypes: GO:0106061, negative regulation of G2/MI transition of meiotic cell cycle [GO:0110031], GO:1902103 Relationships: is a type of negative regulation of meiotic cell cycle [GO:0051447]; is a type of negative regulation of cell cycle phase transition [GO:1901988]; is a type of regulation of meiotic cell cycle phase transition [GO:1901993]; negatively regulates meiotic cell cycle phase transition [GO:0044771] References: PMID:22841721 Sources: GOC:TermGenie, GOC:mtg_cell_cycle